lateral growth [GO:0080190] (BP) Sources: PO:0020145 Relationships: is a type of GO:0040007 Subtypes: secondary growth [GO:0080117], secondary thickening [GO:0080191], GO:0080192, diffuse secondary thickening [GO:0080193] Note: Includes thickening of plant axes (PO:0025004) due to the activity of a cambium (PO:0005597), known as secondary growth and found in most gymnosperms and dicotyledons, a primary thickening meristem (PO:0005039) as found in many monocotyledons, some ferns and some cycads, or secondary thickening meristem, (PO:0025414) as found in some monocotyledons. Definition: Growth of a plant axis (shoot axis or root) that originates from a lateral meristem.